positive regulation of iron-sulfur-molybdenum cofactor assembly [GO:1900508] (biological process) Sources: GOC:TermGenie, GOC:mengo_curators Also known as: activation of FeMoco assembly, activation of FeMoco biosynthetic process, activation of iron molybdenum cofactor assembly, activation of iron molybdenum cofactor biosynthesis, activation of iron molybdenum cofactor biosynthetic process, positive regulation of FeMoco assembly, positive regulation of FeMoco biosynthetic process, positive regulation of iron molybdenum cofactor assembly, positive regulation of iron molybdenum cofactor biosynthesis, positive regulation of iron molybdenum cofactor biosynthetic process, up regulation of FeMoco assembly, up regulation of FeMoco biosynthetic process, up regulation of iron molybdenum cofactor assembly, up regulation of iron molybdenum cofactor biosynthesis, up regulation of iron molybdenum cofactor biosynthetic process, up regulation of iron-sulfur-molybdenum cofactor assembly, up-regulation of FeMoco assembly, up-regulation of FeMoco biosynthetic process, up-regulation of iron molybdenum cofactor assembly, up-regulation of iron molybdenum cofactor biosynthesis, up-regulation of iron molybdenum cofactor biosynthetic process, up-regulation of iron-sulfur-molybdenum cofactor assembly, upregulation of FeMoco assembly, upregulation of FeMoco biosynthetic process, upregulation of iron molybdenum cofactor assembly, upregulation of iron molybdenum cofactor biosynthesis, upregulation of iron molybdenum cofactor biosynthetic process, upregulation of iron-sulfur-molybdenum cofactor assembly, activation of iron-sulfur-molybdenum cofactor assembly Definition: Any process that activates or increases the frequency, rate or extent of iron-sulfur-molybdenum cofactor assembly. Relationships: is_a GO:1900506; is a type of GO:1903331; positively regulates iron-sulfur-molybdenum cofactor assembly [GO:0044593]